{
  "term_id": "GO:0005634",
  "gene_name": "Protein artemis",
  "gene": "UniProtKB:Q96SD1",
  "gene_symbol": "DCLRE1C",
  "term_label": "nucleus"
}